purine ribonucleotide catabolic process [GO:0009154] (biological process) Sources: GOC:go_curators, ISBN:0198506732 Also known as: purine ribonucleotide breakdown, purine ribonucleotide catabolism, purine ribonucleotide degradation Subtypes: ITP catabolic process [GO:0006193], AMP catabolic process [GO:0006196], cAMP catabolic process [GO:0006198], IMP catabolic process [GO:0006204], guanosine tetraphosphate catabolic process [GO:0015971], guanosine pentaphosphate catabolic process [GO:0015974], ADP catabolic process [GO:0046032], GMP catabolic process [GO:0046038], cGMP catabolic process [GO:0046069], IDP catabolic process [GO:0046709], GDP catabolic process [GO:0046712], GO:1901911 Definition: The chemical reactions and pathways resulting in the breakdown of a purine ribonucleotide, a compound consisting of ribonucleoside (a purine base linked to a ribose sugar) esterified with a phosphate group at either the 3' or 5'-hydroxyl group of the sugar. Relationships: is a type of purine nucleotide catabolic process [GO:0006195]; is a type of purine ribonucleotide metabolic process [GO:0009150]; is a type of GO:0009261